IgE immunoglobulin complex, circulating [GO:0071743] (cellular component) Note: Note that an IgE immunoglobulin complex has the function of antigen binding if a suitable antigen is available. Definition: A protein complex composed of two identical immunoglobulin heavy chains of the IgE isotype and two identical immunoglobulin light chains, held together by disulfide bonds, and present in the extracellular space, in mucosal areas or other tissues, or circulating in the blood or lymph. Sources: GOC:add, ISBN:0781765196 Also known as: IgE antibody Relationships: is a type of immunoglobulin complex, circulating [GO:0042571]; is a type of GO:0071742